{
  "gene": "UniProtKB:Q00537",
  "gene_symbol": "CDK17",
  "gene_name": "Cyclin-dependent kinase 17",
  "term_label": "regulation of cell cycle phase transition",
  "term_id": "GO:1901987"
}